{
  "term_label": "Unknown molecular function",
  "gene_name": "Cilia- and flagella-associated protein 54",
  "gene_symbol": "CFAP54",
  "term_id": "UNKNOWN:0001",
  "gene": "UniProtKB:Q96N23"
}